right caudal basal body [GO:1902678] (cellular component) Definition: Any ciliary basal body that is part of a right caudal flagellum found in Giardia species (trophozoite stage). References: PMID:16607022, PMID:5961344 Sources: GOC:TermGenie, GOC:giardia, GO_REF:0000064, ISBN:9780124260207 Also known as: cilial basal body of right caudal cilium, cilial basal body of right caudal flagellum, ciliary basal body of right caudal cilium, ciliary basal body of right caudal flagellum, cilium basal body of right caudal cilium, cilium basal body of right caudal flagellum, microtubule basal body of right caudal cilium, microtubule basal body of right caudal flagellum, right caudal flagellum ciliary basal body Note: Note that we deem cilium and microtubule-based flagellum to be equivalent. Also note that, due to the asymmetric nature of the Giardia trophozoite, this term is defined spatially as the trophozoite is viewed from the dorsal side, with the two nuclei dorsal to the ventral disc, and the ventral disc toward the anterior. Relationships: is a type of ciliary basal body [GO:0036064]; is part of right caudal flagellum [GO:0097561]